mammary gland epithelium development [GO:0061180] (BP) Relationships: is a type of epithelium development [GO:0060429]; is part of mammary gland development [GO:0030879] Definition: The process whose specific outcome is the progression of the mammary gland epithelium over time, from its formation to the mature structure. The mammary gland is a large compound sebaceous gland that in female mammals is modified to secrete milk. Also known as: breast epithelium development Sources: GOC:dph, GOC:yaf